{
  "term_id": "GO:0007166",
  "term_label": "cell surface receptor signaling pathway",
  "gene_name": "Probable non-functional T cell receptor beta variable 5-7",
  "gene_symbol": "TRBV5-7",
  "gene": "UniProtKB:A0A0A0MS05"
}